{
  "term_label": "nucleolus",
  "term_id": "GO:0005730",
  "gene_symbol": "NOL8",
  "gene_name": "Nucleolar protein 8",
  "gene": "UniProtKB:Q76FK4"
}